{
  "gene_symbol": "RAB11FIP5",
  "term_id": "UNKNOWN:0001",
  "gene": "UniProtKB:Q9BXF6",
  "term_label": "Unknown molecular function",
  "gene_name": "Rab11 family-interacting protein 5"
}